{
  "term_id": "GO:0016567",
  "gene_symbol": "CDC27",
  "gene_name": "Cell division cycle protein 27 homolog",
  "term_label": "protein ubiquitination",
  "gene": "UniProtKB:P30260"
}